indole-3-glycerol-phosphate lyase activity [GO:0033984] (molecular function) Definition: Catalysis of the reaction: (1S,2R)-1-C-(indol-3-yl)glycerol 3-phosphate = indole + D-glyceraldehyde 3-phosphate. Sources: EC:4.1.2.8 Also known as: tryptophan synthase alpha activity, tryptophan synthase alpha subunit activity, (1S,2R)-1-C-(indol-3-yl)glycerol 3-phosphate D-glyceraldehyde-3-phosphate-lyase (indole-forming) activity, (1S,2R)-1-C-(indol-3-yl)glycerol 3-phosphate D-glyceraldehyde-3-phosphate-lyase activity, BX1, IGL, TSA, indole glycerol phosphate hydrolase activity, indole synthase activity, indole-3-glycerol phosphate lyase activity, indole-3-glycerolphosphate D-glyceraldehyde-3-phosphate-lyase activity, indoleglycerolphosphate aldolase activity Relationships: is a type of aldehyde-lyase activity [GO:0016832]